colon epithelial cell migration [GO:0061580] (biological process) Sources: GOC:dph Subtypes: colon epithelial cell chemotaxis [GO:0061583] Relationships: is a type of intestinal epithelial cell migration [GO:0061582] Definition: The orderly movement of a colonic epithelial cell from one site to another, often during the development of a multicellular organism.